{
  "gene": "UniProtKB:Q96IW7",
  "term_id": "UNKNOWN:0001",
  "term_label": "Unknown molecular function",
  "gene_name": "Vesicle-trafficking protein SEC22a",
  "gene_symbol": "SEC22A"
}